{
  "term_label": "inositol-1,4,5-trisphosphate 3-kinase activity",
  "term_id": "GO:0008440",
  "gene": "UniProtKB:Q8NFU5",
  "gene_name": "Inositol polyphosphate multikinase",
  "gene_symbol": "IPMK"
}